{
  "gene_symbol": "CAT",
  "term_id": "GO:0042744",
  "gene_name": "Catalase",
  "term_label": "hydrogen peroxide catabolic process",
  "gene": "UniProtKB:P04040"
}